phagocytosis, engulfment [GO:0006911] (biological process) Definition: The internalization of bacteria, immune complexes and other particulate matter or of an apoptotic cell by phagocytosis, including the membrane and cytoskeletal processes required, which involves one of three mechanisms: zippering of pseudopods around a target via repeated receptor-ligand interactions, sinking of the target directly into plasma membrane of the phagocytosing cell, or induced uptake via an enhanced membrane ruffling of the phagocytosing cell similar to macropinocytosis. Sources: GOC:curators, ISBN:0781735149 Also known as: phagosome biosynthesis, phagosome formation Relationships: is a type of plasma membrane invagination [GO:0099024]; is part of phagocytosis [GO:0006909] Subtypes: GO:0043652 Regulation: regulated by regulation of phagocytosis, engulfment [GO:0060099]; positively regulated by positive regulation of phagocytosis, engulfment [GO:0060100]; negatively regulated by GO:0060101